very long-chain fatty acid-CoA ligase activity [GO:0031957] (molecular function) Note: While there is not universal consensus on the lengths of short-, medium-, long- and very-long-chain fatty acids, the GO uses the definitions in ChEBI (see CHEBI:26666, CHEBI:59554, CHEBI:15904 and CHEBI:27283). References: PMID:18024425 Sources: RHEA:54536 Definition: Catalysis of the reaction: a very long-chain fatty acid + ATP + CoA = a very long-chain fatty acyl-CoA + AMP + diphosphate. A very long-chain fatty acid has an aliphatic tail containing more than 22 carbons. Relationships: is a type of fatty acid-CoA ligase activity [GO:0120515] Also known as: very-long-chain fatty acid-CoA ligase activity, very-long-chain-fatty-acid-CoA ligase activity, very-long-chain fatty acid activation